{
  "gene_name": "Rho GTPase-activating protein 10",
  "gene_symbol": "ARHGAP10",
  "term_label": "negative regulation of apoptotic process",
  "gene": "UniProtKB:A1A4S6",
  "term_id": "GO:0043066"
}